{
  "gene_symbol": "RHEX",
  "gene": "UniProtKB:Q6ZWK4",
  "term_id": "UNKNOWN:0002",
  "term_label": "Unknown biological process",
  "gene_name": "Regulator of hemoglobinization and erythroid cell expansion protein"
}